transition between slow and fast fiber [GO:0014886] (BP) Sources: GOC:ef, GOC:mtg_muscle Also known as: transition between slow and fast fibre, transition slow-fast fiber, transition slow-fast fibre Relationships: is a type of regulation of skeletal muscle adaptation [GO:0014733] Definition: The process of conversion of slow-contracting muscle fibers to a faster character. This may involve increasing of contractile rate, fast myosin gene induction, increase in glycolytic metabolic properties, altered electrophysiology and altered innervation. This process also regulates skeletal muscle adapatation.